4-methylthiopropyl glucosinolate S-oxygenase activity [GO:0080103] (molecular function) Definition: Catalysis of the reaction: 4-methylthiopropyl-glucosinolate = 4-methylsulfinylpropyl-glucosinolate. References: PMID:18799661 Relationships: is a type of oxidoreductase activity, acting on paired donors, with incorporation or reduction of molecular oxygen [GO:0016705]